{
  "gene_symbol": "SFRP2",
  "gene_name": "Secreted frizzled-related protein 2",
  "gene": "UniProtKB:Q96HF1",
  "term_label": "Wnt-protein binding",
  "term_id": "GO:0017147"
}